pathogen-derived receptor ligand activity [GO:0140295] (molecular function) Definition: The activity of a pathogen-derived entity that interacts with a host receptor to activate effector-triggered immunity. References: PMID:20601497 Also known as: host-selective toxin, innate receptor ligand activity, necrotrophic effector Note: Note that this term is meant to annotate effectors for which the evolved activity is to act as a ligand to activate (for necrotrophs) or suppress (for biotrophs) the host immune system. It should not be used to annotate PAMPs (pathogen-associated molecular pattern molecules) or similar types of microbial proteins recognized by the host innate immune system (for example, PAMPs are recognized by toll-like receptors (TLRs) and other pattern recognition receptors (PRRs) in both plants and animals). PAMPs activate innate immune responses, protecting the host from infection, but this is not the molecular function of PAMPs; those usually form the structure of the bacterial cell wall. Relationships: is a type of receptor ligand activity [GO:0048018]